{
  "gene_name": "Tripartite motif-containing protein 5",
  "gene_symbol": "TRIM5",
  "term_id": "GO:0045087",
  "term_label": "innate immune response",
  "gene": "UniProtKB:Q9C035"
}